RNA cap 4 binding [GO:0000342] (molecular function) Relationships: is a type of RNA cap binding [GO:0000339] Definition: Binding to a hypermethylated cap structure consisting of 7-methylguanosine (m(7)G) followed by four methylated nucleotides (cap 4): 7-methylguanosine-ppp-N6, N6, 2'-O-trimethyladenosine-p-2'-O-methyladenosine-p-2'-O-methylcytosine-p-N3, 2'-O-dimethyluridine Such caps are known to be found at the 5' ends of SL RNAs of trypanosomatid protozoa. References: PMID:10880518, PMID:12121975 Sources: GOC:krc